{
  "gene_symbol": "MYH9",
  "gene_name": "Myosin-9",
  "term_id": "GO:0005737",
  "term_label": "cytoplasm",
  "gene": "UniProtKB:P35579"
}